{
  "gene": "UniProtKB:O60568",
  "gene_name": "Multifunctional procollagen lysine hydroxylase and glycosyltransferase LH3",
  "gene_symbol": "PLOD3",
  "term_label": "procollagen-lysine 5-dioxygenase activity",
  "term_id": "GO:0008475"
}